vasoconstriction of artery involved in aortic body chemoreceptor response to lowering of systemic arterial blood pressure [GO:0003043] (biological process) Relationships: is a type of GO:0002012; BFO_0000050 regulation of systemic arterial blood pressure by aortic body chemoreceptor signaling [GO:0003028] Sources: GOC:mtg_cardio Definition: A process that is triggered by aortic body-vasomotor excitation and results in a decrease in the diameter of an artery during the chemoreceptor response to decreased blood pressure. Also known as: vasoconstriction of artery during aortic body chemoreceptor response to lowering of systemic arterial blood pressure